{
  "gene_symbol": "TGFBR2",
  "gene": "UniProtKB:P37173",
  "gene_name": "TGF-beta receptor type-2",
  "term_id": "GO:0048179",
  "term_label": "activin receptor complex"
}